{
  "term_id": "UNKNOWN:0002",
  "gene_name": "Putative uncharacterized protein encoded by LINC00301",
  "gene": "UniProtKB:Q8NCQ3",
  "gene_symbol": "LINC00301",
  "term_label": "Unknown biological process"
}